{
  "gene": "UniProtKB:O43315",
  "term_label": "water transport",
  "gene_symbol": "AQP9",
  "gene_name": "Aquaporin-9",
  "term_id": "GO:0006833"
}